{
  "gene_name": "Phosphoenolpyruvate carboxykinase [GTP], mitochondrial",
  "term_label": "mitochondrial matrix",
  "gene": "UniProtKB:Q16822",
  "term_id": "GO:0005759",
  "gene_symbol": "PCK2"
}